 [go#goslim:aspergillus] Note: Aspergillus GO slim